prospore contractile ring [GO:0032157] (cellular component) Definition: A contractile ring, i.e. a cytoskeletal structure composed of actin filaments and myosin, that forms beneath the plasma membrane of the prospore envelope in meiotic cells in preparation for completing cytokinesis. Relationships: is a type of meiotic actomyosin contractile ring [GO:0110086]; is part of GO:0042764 Also known as: actomyosin ring, cytokinetic ring, meiotic contractile ring References: PMID:16009555 Sources: GOC:krc